pattern orientation [GO:0007633] (biological process) Definition: The actions or reactions of an individual in response to the orientation of a visual pattern. This is exemplified by some classes of insects which are able to detect and learn the orientation of a set of stripes and subsequently behaviorally discriminate between horizontal, vertical or 45 degree stripes. Also known as: behavioral response to pattern orientation, behavioural response to pattern orientation Relationships: is a type of visual behavior [GO:0007632] References: PMID:9933535 Sources: GOC:jid